nucleotide-binding domain, leucine rich repeat containing receptor signaling pathway [GO:0035872] (biological process) References: PMID:18280719, PMID:32838963, PMID:36973360 Sources: GOC:sj Definition: The series of molecular signals initiated by a ligand binding to a nucleotide-binding domain, leucine rich repeat containing receptor (NLR), and ending with the regulation of a downstream cellular process. NLRs are cytoplasmic receptors defined by their tripartite domain architecture that contains: a variable C-terminus, a middle nucleotide-binding domain, and a LRR domain that is variable in the repeats composition and number. Also known as: NLR signaling pathway, nucleotide-binding domain leucine-rich repeat containing receptor signaling pathway, nucleotide-binding domain, leucine rich repeat containing receptor signal transduction, nucleotide-binding domain, leucine rich repeat containing receptor signal transduction pathway, nucleotide-binding domain, leucine rich repeat containing receptor signalling pathway, NOD-like receptor signaling pathway Relationships: is a type of GO:0002753 Regulation: regulated by regulation of nucleotide-binding domain, leucine rich repeat containing receptor signaling pathway [GO:0070424]; negatively regulated by negative regulation of nucleotide-binding domain, leucine rich repeat containing receptor signaling pathway [GO:0070425]; positively regulated by GO:0070426 Subtypes: GO:0070427, nucleotide-binding oligomerization domain containing 2 signaling pathway [GO:0070431]